{
  "gene_symbol": "GNA14",
  "term_id": "GO:0007188",
  "term_label": "adenylate cyclase-modulating G protein-coupled receptor signaling pathway",
  "gene": "UniProtKB:O95837",
  "gene_name": "Guanine nucleotide-binding protein subunit alpha-14"
}